{
  "term_id": "GO:0050852",
  "term_label": "T cell receptor signaling pathway",
  "gene_name": "Mucosa-associated lymphoid tissue lymphoma translocation protein 1",
  "gene": "UniProtKB:Q9UDY8",
  "gene_symbol": "MALT1"
}